{
  "gene_name": "Guanine nucleotide-binding protein G(I)_G(S)_G(O) subunit gamma-2",
  "term_id": "GO:0005834",
  "gene_symbol": "GNG2",
  "gene": "UniProtKB:P59768",
  "term_label": "heterotrimeric G-protein complex"
}